metanephric long descending thin limb bend development [GO:0072226] (biological process) Definition: The process whose specific outcome is the progression of the metanephric long descending thin limb bend over time, from its formation to the mature structure. The metanephric long descending thin limb bend is a part of the descending thin limb of a long nephron that lies beyond the prebend segment in the metanephros. Relationships: is a type of long descending thin limb bend development [GO:0072065]; is part of metanephric descending thin limb development [GO:0072220]; is part of GO:0072269 Sources: GOC:mtg_kidney_jan10